{
  "term_id": "GO:0000981",
  "gene_symbol": "TFAP4",
  "term_label": "DNA-binding transcription factor activity, RNA polymerase II-specific",
  "gene": "UniProtKB:Q01664",
  "gene_name": "Transcription factor AP-4"
}